{
  "gene_symbol": "TBX4",
  "gene_name": "T-box transcription factor TBX4",
  "gene": "UniProtKB:P57082",
  "term_id": "GO:0001708",
  "term_label": "cell fate specification"
}